Rho GDP-dissociation inhibitor activity [GO:0005094] (molecular function) Relationships: is a type of GDP-dissociation inhibitor activity [GO:0005092] Definition: Prevents the dissociation of GDP from the small GTPase Rho, thereby preventing GTP from binding. Sources: GOC:mah